{
  "gene_name": "Plasmanylethanolamine desaturase 1",
  "term_label": "ether lipid biosynthetic process",
  "gene_symbol": "PEDS1",
  "term_id": "GO:0008611",
  "gene": "UniProtKB:A5PLL7"
}